{
  "term_id": "GO:0098793",
  "gene_name": "Huntingtin-interacting protein 1",
  "gene": "UniProtKB:O00291",
  "gene_symbol": "HIP1",
  "term_label": "presynapse"
}